{
  "gene": "UniProtKB:Q9UKN1",
  "term_label": "Unknown cellular component",
  "gene_name": "Mucin-12",
  "term_id": "UNKNOWN:0003",
  "gene_symbol": "MUC12"
}